negative regulation of response to type II interferon [GO:0060331] (biological process) Subtypes: GO:0060336 Sources: GOC:dph Definition: Any process that decreases the rate, frequency or extent of a response to type II interferon (interferon-gamma). Response to interferon gamma is a change in state or activity of a cell or an organism (in terms of movement, secretion, enzyme production, gene expression, etc.) as a result of an interferon-gamma stimulus. Relationships: is a type of negative regulation of innate immune response [GO:0045824]; is a type of GO:0060330; is a type of negative regulation of response to cytokine stimulus [GO:0060761]; negatively regulates GO:0034341 Also known as: negative regulation of response to type II IFN, negative regulation of response to immune interferon, negative regulation of response to interferon-gamma, negative regulation of response to gamma-interferon